{
  "gene_name": "Flavin-containing monooxygenase 3",
  "gene": "UniProtKB:P31513",
  "gene_symbol": "FMO3",
  "term_label": "taurine biosynthetic process",
  "term_id": "GO:0042412"
}